{
  "term_id": "GO:0007399",
  "gene": "UniProtKB:Q92752",
  "gene_name": "Tenascin-R",
  "gene_symbol": "TNR",
  "term_label": "nervous system development"
}